{
  "gene": "UniProtKB:O95045",
  "term_id": "GO:0005829",
  "term_label": "cytosol",
  "gene_name": "Uridine phosphorylase 2",
  "gene_symbol": "UPP2"
}